{
  "gene_name": "Diablo IAP-binding mitochondrial protein",
  "term_label": "Unknown molecular function",
  "gene_symbol": "DIABLO",
  "gene": "UniProtKB:Q9NR28",
  "term_id": "UNKNOWN:0001"
}